{
  "gene_name": "2-amino-3-carboxymuconate-6-semialdehyde decarboxylase",
  "term_label": "secondary metabolic process",
  "gene_symbol": "ACMSD",
  "term_id": "GO:0019748",
  "gene": "UniProtKB:Q8TDX5"
}